{
  "gene_name": "TBC1 domain family member 14",
  "term_label": "recycling endosome",
  "gene_symbol": "TBC1D14",
  "term_id": "GO:0055037",
  "gene": "UniProtKB:Q9P2M4"
}